glyoxylate cycle [GO:0006097] (BP) Definition: A modification of the TCA cycle occurring in some plants and microorganisms, in which isocitrate is cleaved to glyoxylate and succinate. Glyoxylate can then react with acetyl-CoA to form malate. Regulation: regulated by regulation of glyoxylate cycle [GO:2000874]; negatively regulated by negative regulation of glyoxylate cycle [GO:2000875]; positively regulated by positive regulation of glyoxylate cycle [GO:2000876] Also known as: glyoxylate bypass Sources: ISBN:0198506732 Relationships: is a type of carbohydrate metabolic process [GO:0005975]; is a type of glyoxylate metabolic process [GO:0046487]